conus arteriosus morphogenesis [GO:0003239] (biological process) Relationships: is a type of cardiac chamber morphogenesis [GO:0003206]; is part of GO:0003238 Definition: The process in which the conus arteriosus is generated and organized. The conus arteriosus is a valved chamber with thick muscular walls stemming from the ventricle and connecting to the pulmonary trunk. Sources: GOC:mtg_heart